{
  "gene_name": "Ras and EF-hand domain-containing protein",
  "term_id": "GO:0019003",
  "gene_symbol": "RASEF",
  "term_label": "GDP binding",
  "gene": "UniProtKB:Q8IZ41"
}